endopeptidase inhibitor activity [GO:0004866] (molecular function) Also known as: endoproteinase inhibitor, proteinase inhibitor, alpha-2 macroglobulin Subtypes: serine-type endopeptidase inhibitor activity [GO:0004867], cysteine-type endopeptidase inhibitor activity [GO:0004869], metalloendopeptidase inhibitor activity [GO:0008191], GO:0019828 Relationships: is a type of peptidase inhibitor activity [GO:0030414]; is a type of endopeptidase regulator activity [GO:0061135]; negatively regulates endopeptidase activity [GO:0004175] Definition: Binds to and stops, prevents or reduces the activity of an endopeptidase. Sources: GOC:jl